{
  "gene_symbol": "RIPK1",
  "term_id": "GO:0097527",
  "gene_name": "Receptor-interacting serine_threonine-protein kinase 1",
  "term_label": "necroptotic signaling pathway",
  "gene": "UniProtKB:Q13546"
}